{
  "gene_symbol": "IRF7",
  "term_label": "regulation of transcription by RNA polymerase II",
  "gene_name": "Interferon regulatory factor 7",
  "term_id": "GO:0006357",
  "gene": "UniProtKB:Q92985"
}